cardiac glial cell development [GO:0060952] (biological process) Sources: GOC:mtg_heart Definition: The process aimed at the progression of a cardiac glial cell over time, from its formation to the fully functional mature cell. Subtypes: neural crest-derived cardiac glial cell development [GO:0060954] Relationships: is a type of GO:0021782; is a type of GO:0055006; is part of cardiac glial cell differentiation [GO:0060950]